kaempferol 3-O-methyltransferase activity [GO:0102449] (MF) Definition: Catalysis of the reaction: kaempferol + S-adenosyl-L-methionine = 3-O-methylkaempferol + H+ + S-adenosyl-L-homocysteine. Sources: RHEA:74743 Relationships: is a type of methyltransferase activity [GO:0008168]